{
  "gene_symbol": "TLN1",
  "term_id": "GO:0030036",
  "gene": "UniProtKB:Q9Y490",
  "term_label": "actin cytoskeleton organization",
  "gene_name": "Talin-1"
}